{
  "term_label": "alpha-tubulin binding",
  "gene_symbol": "EFHC1",
  "term_id": "GO:0043014",
  "gene": "UniProtKB:Q5JVL4",
  "gene_name": "EF-hand domain-containing protein 1"
}